{
  "gene": "UniProtKB:P56715",
  "term_id": "GO:0005930",
  "gene_symbol": "RP1",
  "term_label": "axoneme",
  "gene_name": "Oxygen-regulated protein 1"
}